{
  "term_label": "water channel activity",
  "gene": "UniProtKB:A0A075B734",
  "gene_symbol": "AQP7B",
  "term_id": "GO:0015250",
  "gene_name": "Aquaporin-7B"
}